{
  "gene_symbol": "CPVL",
  "term_label": "Unknown biological process",
  "gene_name": "Probable serine carboxypeptidase CPVL",
  "gene": "UniProtKB:Q9H3G5",
  "term_id": "UNKNOWN:0002"
}